P-TEFb-cap methyltransferase complex [GO:0070693] (CC) Definition: A protein complex that is formed by the association of positive transcription elongation factor complex b (P-TEFb) with the mRNA capping methyltransferase. References: PMID:17332744, PMID:19328067 Relationships: is a type of nuclear protein-containing complex [GO:0140513] Also known as: Cdk9-Pcm1 complex, P-TEFb-Pcm1 complex